{
  "term_label": "Unknown biological process",
  "gene_symbol": "STIP1",
  "gene_name": "Stress-induced-phosphoprotein 1",
  "term_id": "UNKNOWN:0002",
  "gene": "UniProtKB:P31948"
}